{
  "term_id": "GO:0017136",
  "term_label": "histone deacetylase activity, NAD-dependent",
  "gene_name": "NAD-dependent protein deacetylase sirtuin-3, mitochondrial",
  "gene": "UniProtKB:Q9NTG7",
  "gene_symbol": "SIRT3"
}